fructan beta-(2,6)-fructosidase activity [GO:0033949] (molecular function) Sources: EC:3.2.1.154 Also known as: 6-FEH, beta-(2,6)-D-fructan fructohydrolase activity, beta-(2,6)-fructan exohydrolase activity Definition: Catalysis of the hydrolysis of terminal, non-reducing (2->6) linked beta-D-fructofuranose residues in fructans. Relationships: is a type of hydrolase activity, hydrolyzing O-glycosyl compounds [GO:0004553]